{
  "gene_name": "Kinetochore-associated protein 1",
  "term_id": "GO:0007094",
  "gene_symbol": "KNTC1",
  "gene": "UniProtKB:P50748",
  "term_label": "mitotic spindle assembly checkpoint signaling"
}